biotin import across plasma membrane [GO:1905135] (biological process) Relationships: is a type of biotin transport [GO:0015878]; is a type of vitamin transmembrane transport [GO:0035461]; is a type of GO:0098739; is a type of carboxylic acid transmembrane transport [GO:1905039] References: PMID:12557275 Sources: GOC:TermGenie, GO_REF:0000075 Also known as: biotin import into cell, biotin import Definition: The directed movement of biotin from outside of a cell, across the plasma membrane and into the cytosol.